{
  "term_id": "GO:0004674",
  "gene_name": "3-phosphoinositide-dependent protein kinase 1",
  "gene": "UniProtKB:O15530",
  "term_label": "protein serine/threonine kinase activity",
  "gene_symbol": "PDPK1"
}